{
  "gene_name": "Nocturnin",
  "gene_symbol": "NOCT",
  "term_label": "Unknown cellular component",
  "term_id": "UNKNOWN:0003",
  "gene": "UniProtKB:Q9UK39"
}